{
  "term_id": "UNKNOWN:0001",
  "gene_name": "Tetratricopeptide repeat protein 27",
  "term_label": "Unknown molecular function",
  "gene": "UniProtKB:Q6P3X3",
  "gene_symbol": "TTC27"
}